{
  "term_label": "Golgi organization",
  "gene": "UniProtKB:Q9H4A6",
  "term_id": "GO:0007030",
  "gene_symbol": "GOLPH3",
  "gene_name": "Golgi phosphoprotein 3"
}